{
  "term_id": "UNKNOWN:0001",
  "gene": "UniProtKB:O95460",
  "gene_name": "Matrilin-4",
  "term_label": "Unknown molecular function",
  "gene_symbol": "MATN4"
}